{
  "term_label": "protein K63-linked ubiquitination",
  "term_id": "GO:0070534",
  "gene": "UniProtKB:Q13404",
  "gene_name": "Ubiquitin-conjugating enzyme E2 variant 1",
  "gene_symbol": "UBE2V1"
}